{
  "term_id": "GO:0043240",
  "gene_symbol": "FANCA",
  "term_label": "Fanconi anaemia nuclear complex",
  "gene": "UniProtKB:O15360",
  "gene_name": "Fanconi anemia group A protein"
}